{
  "gene_name": "Melanocortin-2 receptor accessory protein 2",
  "term_label": "type 3 melanocortin receptor binding",
  "term_id": "GO:0031781",
  "gene": "UniProtKB:Q96G30",
  "gene_symbol": "MRAP2"
}